{
  "gene_name": "Endothelial PAS domain-containing protein 1",
  "term_id": "GO:0005634",
  "gene_symbol": "EPAS1",
  "gene": "UniProtKB:Q99814",
  "term_label": "nucleus"
}